{
  "term_label": "DNA-binding transcription factor activity, RNA polymerase II-specific",
  "gene_name": "Hairy_enhancer-of-split related with YRPW motif-like protein",
  "gene": "UniProtKB:Q9NQ87",
  "term_id": "GO:0000981",
  "gene_symbol": "HEYL"
}